{
  "gene": "UniProtKB:Q14008",
  "term_id": "GO:0030951",
  "term_label": "establishment or maintenance of microtubule cytoskeleton polarity",
  "gene_symbol": "CKAP5",
  "gene_name": "Cytoskeleton-associated protein 5"
}